{
  "gene": "UniProtKB:P0DKB5",
  "gene_symbol": "TPBGL",
  "term_label": "Unknown molecular function",
  "term_id": "UNKNOWN:0001",
  "gene_name": "Trophoblast glycoprotein-like"
}